{
  "gene_symbol": "CEP170",
  "term_label": "Unknown biological process",
  "term_id": "UNKNOWN:0002",
  "gene": "UniProtKB:Q5SW79",
  "gene_name": "Centrosomal protein of 170 kDa"
}